{
  "gene_name": "Vitamin D-binding protein",
  "gene": "UniProtKB:P02774",
  "term_id": "GO:0031667",
  "term_label": "response to nutrient levels",
  "gene_symbol": "GC"
}